{
  "term_label": "plasma membrane",
  "gene_name": "Protocadherin-9",
  "gene": "UniProtKB:Q9HC56",
  "gene_symbol": "PCDH9",
  "term_id": "GO:0005886"
}